{
  "gene_name": "Semaphorin-4A",
  "term_id": "GO:0050919",
  "term_label": "negative chemotaxis",
  "gene_symbol": "SEMA4A",
  "gene": "UniProtKB:Q9H3S1"
}